{
  "gene_symbol": "BCAN",
  "term_id": "GO:0001501",
  "gene_name": "Brevican core protein",
  "gene": "UniProtKB:Q96GW7",
  "term_label": "skeletal system development"
}